positive regulation of protein kinase C signaling [GO:0090037] (biological process) Also known as: positive regulation of protein kinase C signalling cascade, positive regulation of protein kinase C signaling cascade Relationships: is a type of regulation of protein kinase C signaling [GO:0090036]; is a type of positive regulation of intracellular signal transduction [GO:1902533]; positively regulates protein kinase C signaling [GO:0070528] Sources: GOC:dph, GOC:tb Definition: Any process that increases the frequency, rate, or extent of a series of reactions, mediated by the intracellular serine/threonine kinase protein kinase C, which occurs as a result of a single trigger reaction or compound.